{
  "term_label": "potassium ion transmembrane transport",
  "term_id": "GO:0071805",
  "gene": "UniProtKB:P57789",
  "gene_symbol": "KCNK10",
  "gene_name": "Potassium channel subfamily K member 10"
}